{
  "term_label": "negative regulation of cell-cell adhesion",
  "term_id": "GO:0022408",
  "gene_symbol": "MUC21",
  "gene_name": "Mucin-21",
  "gene": "UniProtKB:Q5SSG8"
}